{
  "gene_name": "NHS-like protein 1",
  "gene_symbol": "NHSL1",
  "term_label": "Unknown cellular component",
  "gene": "UniProtKB:Q5SYE7",
  "term_id": "UNKNOWN:0003"
}